{
  "gene_symbol": "RNF8",
  "term_label": "protein K48-linked ubiquitination",
  "gene": "UniProtKB:O76064",
  "term_id": "GO:0070936",
  "gene_name": "E3 ubiquitin-protein ligase RNF8"
}